{
  "term_id": "GO:0004467",
  "gene": "UniProtKB:Q5FVE4",
  "term_label": "long-chain fatty acid-CoA ligase activity",
  "gene_name": "Long-chain-fatty-acid--CoA ligase ACSBG2",
  "gene_symbol": "ACSBG2"
}